{
  "gene_name": "Thymidine phosphorylase",
  "gene_symbol": "TYMP",
  "term_label": "cytosol",
  "term_id": "GO:0005829",
  "gene": "UniProtKB:P19971"
}